{
  "gene": "UniProtKB:Q8IW52",
  "gene_name": "SLIT and NTRK-like protein 4",
  "term_label": "Unknown molecular function",
  "gene_symbol": "SLITRK4",
  "term_id": "UNKNOWN:0001"
}